molybdopterin cofactor biosynthetic process [GO:0032324] (biological process) Subtypes: Mo-molybdopterin cofactor biosynthetic process [GO:0006777], W-molybdopterin cofactor biosynthetic process [GO:0042047] Also known as: molybdopterin cofactor anabolism, molybdopterin cofactor synthesis, molybdopterin cofactor biosynthesis, molybdopterin cofactor formation Sources: GOC:mah Relationships: is a type of molybdopterin cofactor metabolic process [GO:0043545]; is a type of organophosphate biosynthetic process [GO:0090407]; BFO_0000051 GO:0030366; has part cysteine desulfurase activity [GO:0031071]; has part molybdopterin adenylyltransferase activity [GO:0061598]; BFO_0000051 molybdopterin-synthase sulfurtransferase activity [GO:0061604]; has part molybdopterin-synthase adenylyltransferase activity [GO:0061605] Definition: The chemical reactions and pathways resulting in the formation of the molybdopterin cofactor (Moco), essential for the catalytic activity of some enzymes, e.g. sulfite oxidase, xanthine dehydrogenase, and aldehyde oxidase. The cofactor consists of a mononuclear molybdenum (Mo-molybdopterin) or tungsten ion (W-molybdopterin) coordinated by one or two molybdopterin ligands.